positive regulation of backward locomotion [GO:1905852] (biological process) Definition: Any process that activates or increases the frequency, rate or extent of backward locomotion. Also known as: up regulation of backward locomotion, up-regulation of backward locomotion, upregulation of backward locomotion, activation of backward locomotion References: PMID:11717360 Sources: GOC:TermGenie, GO_REF:0000058 Relationships: is a type of positive regulation of locomotion [GO:0040017]; is a type of GO:0043058; positively regulates backward locomotion [GO:0043057]